{
  "gene_name": "Large ribosomal subunit protein mL55",
  "gene_symbol": "MRPL55",
  "term_label": "structural constituent of ribosome",
  "gene": "UniProtKB:Q7Z7F7",
  "term_id": "GO:0003735"
}